{
  "gene": "UniProtKB:P41212",
  "term_label": "DNA-binding transcription factor activity, RNA polymerase II-specific",
  "term_id": "GO:0000981",
  "gene_name": "Transcription factor ETV6",
  "gene_symbol": "ETV6"
}